{
  "term_id": "GO:0015126",
  "term_label": "canalicular bile acid transmembrane transporter activity",
  "gene_name": "Bile salt export pump",
  "gene": "UniProtKB:O95342",
  "gene_symbol": "ABCB11"
}